{
  "term_label": "plasma membrane",
  "gene_name": "Olfactory receptor 2H1",
  "gene": "UniProtKB:Q9GZK4",
  "term_id": "GO:0005886",
  "gene_symbol": "OR2H1"
}